{
  "term_id": "GO:0050870",
  "term_label": "positive regulation of T cell activation",
  "gene": "UniProtKB:Q30154",
  "gene_symbol": "HLA-DRB5",
  "gene_name": "HLA class II histocompatibility antigen, DR beta 5 chain"
}